negative regulation of stomach neuroendocrine cell differentiation [GO:0061106] (biological process) Sources: GOC:dph Definition: Any process that decreases the rate, frequency or extent of the differentiation of a neuroendocrine cell in the stomach. Relationships: is a type of inhibition of neuroepithelial cell differentiation [GO:0002085]; is a type of negative regulation of neuron differentiation [GO:0045665]; is a type of regulation of stomach neuroendocrine cell differentiation [GO:0061105]; negatively regulates GO:0061102